{
  "gene_symbol": "GGT3P",
  "term_id": "GO:0005886",
  "gene_name": "Putative glutathione hydrolase 3 proenzyme",
  "gene": "UniProtKB:A6NGU5",
  "term_label": "plasma membrane"
}